{
  "gene_symbol": "COX14",
  "term_id": "UNKNOWN:0001",
  "term_label": "Unknown molecular function",
  "gene": "UniProtKB:Q96I36",
  "gene_name": "Cytochrome c oxidase assembly protein COX14"
}